{
  "gene_symbol": "PCYT2",
  "gene_name": "Ethanolamine-phosphate cytidylyltransferase",
  "term_label": "phosphatidylethanolamine biosynthetic process",
  "gene": "UniProtKB:Q99447",
  "term_id": "GO:0006646"
}